{
  "term_id": "UNKNOWN:0002",
  "term_label": "Unknown biological process",
  "gene": "UniProtKB:Q5VVB8",
  "gene_name": "Transmembrane protein 244",
  "gene_symbol": "TMEM244"
}